{
  "gene": "UniProtKB:P21579",
  "term_label": "calcium-dependent activation of synaptic vesicle fusion",
  "term_id": "GO:0099502",
  "gene_symbol": "SYT1",
  "gene_name": "Synaptotagmin-1"
}